regulation of cellooligosaccharide catabolic process [GO:2000963] (biological process) Definition: Any process that modulates the frequency, rate or extent of cellooligosaccharide catabolic process. Relationships: is a type of GO:0043470; RO_0002211 GO:2000903 Subtypes: negative regulation of cellooligosaccharide catabolic process [GO:2000964], GO:2000965 Also known as: regulation of cellooligosaccharide catabolism Sources: GOC:mengo_curators